{
  "gene_symbol": "ADH4",
  "term_label": "alcohol dehydrogenase (NAD+) activity",
  "term_id": "GO:0004022",
  "gene": "UniProtKB:P08319",
  "gene_name": "All-trans-retinol dehydrogenase [NAD(+)] ADH4"
}